D-4-hydroxyphenylglycine transaminase activity [GO:0047320] (molecular function) Relationships: is a type of transaminase activity [GO:0008483] Sources: EC:2.6.1.72, RHEA:15589 Also known as: D-4-hydroxyphenylglycine aminotransferase activity, D-4-hydroxyphenylglycine:2-oxoglutarate aminotransferase activity, D-hydroxyphenylglycine aminotransferase activity Definition: Catalysis of the reaction: 2-oxoglutarate + D-4-hydroxyphenylglycine = 4-hydroxyphenylglyoxylate + L-glutamate.